D-arabinitol 4-dehydrogenase activity [GO:0047813] (molecular function) Definition: Catalysis of the reaction: D-arabinitol + NAD+ = D-xylulose + NADH. Sources: EC:1.1.1.11, MetaCyc:D-ARABINITOL-4-DEHYDROGENASE-RXN Relationships: is a type of oxidoreductase activity, acting on the CH-OH group of donors, NAD or NADP as acceptor [GO:0016616]